{
  "term_label": "Golgi transport complex",
  "gene_name": "Conserved oligomeric Golgi complex subunit 4",
  "gene": "UniProtKB:Q9H9E3",
  "term_id": "GO:0017119",
  "gene_symbol": "COG4"
}